{
  "gene_symbol": "AFTPH",
  "term_label": "Unknown biological process",
  "term_id": "UNKNOWN:0002",
  "gene_name": "Aftiphilin",
  "gene": "UniProtKB:Q6ULP2"
}